postsynaptic density [GO:0014069] (cellular component) References: PMID:14532281 Sources: GOC:BHF, GOC:dos, GOC:ef, GOC:jid, GOC:pr Subtypes: glutamatergic postsynaptic density [GO:0099573] Relationships: is a type of GO:0099572; is part of asymmetric synapse [GO:0032279] Also known as: neuronal postsynaptic density, post synaptic density, post-synaptic density, postsynaptic density of dendrite Definition: An electron dense network of proteins within and adjacent to the postsynaptic membrane of an asymmetric, neuron-neuron synapse. Its major components include neurotransmitter receptors and the proteins that spatially and functionally organize them such as anchoring and scaffolding molecules, signaling enzymes and cytoskeletal components.